{
  "term_label": "Unknown biological process",
  "gene": "UniProtKB:Q9P016",
  "term_id": "UNKNOWN:0002",
  "gene_symbol": "THYN1",
  "gene_name": "Thymocyte nuclear protein 1"
}